{
  "gene_name": "Peptidyl-prolyl cis-trans isomerase A-like 4F",
  "term_label": "cyclosporin A binding",
  "gene_symbol": "PPIAL4F",
  "term_id": "GO:0016018",
  "gene": "UniProtKB:P0DN26"
}